{
  "gene": "UniProtKB:P17098",
  "gene_symbol": "ZNF8",
  "gene_name": "Zinc finger protein 8",
  "term_label": "RNA polymerase II cis-regulatory region sequence-specific DNA binding",
  "term_id": "GO:0000978"
}